{
  "term_id": "UNKNOWN:0002",
  "gene_symbol": "ZFTRAF1",
  "gene_name": "Zinc finger TRAF-type-containing protein 1",
  "term_label": "Unknown biological process",
  "gene": "UniProtKB:P0DTL6"
}